positive regulation of vitamin metabolic process [GO:0046136] (biological process) Sources: GOC:ai Relationships: is a type of regulation of vitamin metabolic process [GO:0030656]; is a type of GO:0062013; positively regulates vitamin metabolic process [GO:0006766] Subtypes: GO:0060557, positive regulation of thiamine biosynthetic process [GO:0090180], GO:1900054, positive regulation of vitamin E biosynthetic process [GO:1904966] Definition: Any process that activates or increases the frequency, rate or extent of the chemical reactions and pathways involving a vitamin, one of a number of unrelated organic substances that occur in many foods in small amounts and that are necessary in trace amounts for the normal metabolic functioning of the body. Also known as: positive regulation of vitamin metabolism, up regulation of vitamin metabolic process, up-regulation of vitamin metabolic process, upregulation of vitamin metabolic process, activation of vitamin metabolic process, stimulation of vitamin metabolic process